{
  "gene_name": "Olfactory receptor 52N4",
  "gene_symbol": "OR52N4",
  "term_label": "Unknown biological process",
  "gene": "UniProtKB:Q8NGI2",
  "term_id": "UNKNOWN:0002"
}